{
  "gene": "UniProtKB:Q9BRP9",
  "term_id": "UNKNOWN:0003",
  "gene_name": "Putative uncharacterized protein MGC13053",
  "term_label": "Unknown cellular component",
  "gene_symbol": "Q9BRP9"
}